{
  "term_id": "GO:0016188",
  "gene_name": "Palmitoyltransferase ZDHHC15",
  "gene_symbol": "ZDHHC15",
  "gene": "UniProtKB:Q96MV8",
  "term_label": "synaptic vesicle maturation"
}